thyroid hormone generation [GO:0006590] (biological process) Sources: GOC:jl, ISBN:0716720094 Relationships: is a type of thyroid hormone metabolic process [GO:0042403] Regulation: regulated by regulation of thyroid hormone generation [GO:2000609]; negatively regulated by negative regulation of thyroid hormone generation [GO:2000610]; positively regulated by positive regulation of thyroid hormone generation [GO:2000611] Definition: The formation of either of the compounds secreted by the thyroid gland, mainly thyroxine and triiodothyronine. This is achieved by the iodination and joining of tyrosine molecules to form the precursor thyroglobin, proteolysis of this precursor gives rise to the thyroid hormones. Note: Note that this term does not fall under the general GO definition for biosynthetic processes, which is 'The chemical reactions and pathways resulting in the formation of... ', because thyroid hormones can only be formed by the proteolysis of a larger molecule (see term definition). The word 'generation' is therefore used in place of biosynthesis.